lipid catabolic process [GO:0016042] (biological process) Also known as: lipid breakdown, lipid catabolism, lipid degradation, lipolysis, multicellular organism lipid catabolic process, multicellular organismal lipid catabolic process Relationships: is a type of lipid metabolic process [GO:0006629]; is a type of GO:0009056 Definition: The chemical reactions and pathways resulting in the breakdown of lipids, compounds soluble in an organic solvent but not, or sparingly, in an aqueous solvent. Regulation: regulated by regulation of lipid catabolic process [GO:0050994]; negatively regulated by GO:0050995; positively regulated by positive regulation of lipid catabolic process [GO:0050996] Subtypes: steroid catabolic process [GO:0006706], isoprenoid catabolic process [GO:0008300], fatty acid catabolic process [GO:0009062], GO:0009104, phospholipid catabolic process [GO:0009395], intestinal lipid catabolic process [GO:0044258], membrane lipid catabolic process [GO:0046466], glycerolipid catabolic process [GO:0046503], cytosolic lipolysis [GO:0061725], emericellamide catabolic process [GO:1900556], fatty acid derivative catabolic process [GO:1901569] Sources: GOC:go_curators